{
  "term_id": "GO:0005024",
  "term_label": "transforming growth factor beta receptor activity",
  "gene_name": "TGF-beta receptor type-2",
  "gene_symbol": "TGFBR2",
  "gene": "UniProtKB:P37173"
}